regulation of circadian rhythm [GO:0042752] (biological process) Definition: Any process that modulates the frequency, rate or extent of a circadian rhythm. A circadian rhythm is a biological process in an organism that recurs with a regularity of approximately 24 hours. Sources: GOC:dph, GOC:jl, GOC:tb Relationships: is_a regulation of biological process [GO:0050789]; regulates circadian rhythm [GO:0007623] Subtypes: entrainment of circadian clock [GO:0009649], GO:0010378, regulation of circadian sleep/wake cycle [GO:0042749], positive regulation of circadian rhythm [GO:0042753], GO:0042754, GO:1904059